negative regulation of inhibin secretion [GO:0032339] (biological process) Also known as: down regulation of inhibin secretion, down-regulation of inhibin secretion, downregulation of inhibin secretion, inhibition of inhibin secretion Sources: GOC:mah Relationships: is a type of regulation of inhibin secretion [GO:0032338]; is a type of negative regulation of hormone secretion [GO:0046888]; is a type of negative regulation of multicellular organismal process [GO:0051241]; RO_0002212 inhibin secretion [GO:0032334] Definition: Any process that stops, prevents, or reduces the frequency, rate or extent of the regulated release of inhibin from a cell.